{
  "gene": "UniProtKB:Q6UUV7",
  "gene_symbol": "CRTC3",
  "term_label": "cytoplasm",
  "gene_name": "CREB-regulated transcription coactivator 3",
  "term_id": "GO:0005737"
}